{
  "gene": "UniProtKB:Q5D1E8",
  "gene_name": "Endoribonuclease ZC3H12A",
  "gene_symbol": "ZC3H12A",
  "term_id": "GO:0036464",
  "term_label": "cytoplasmic ribonucleoprotein granule"
}